{
  "gene_name": "F-box only protein 10",
  "term_id": "GO:0042981",
  "gene": "UniProtKB:Q9UK96",
  "gene_symbol": "FBXO10",
  "term_label": "regulation of apoptotic process"
}